sterigmatocystin biosynthetic process [GO:0045461] (biological process) Definition: The chemical reactions and pathways resulting in the formation of sterigmatocystin, a carcinogenic mycotoxin produced in high yields by strains of the common molds. Also known as: sterigmatocystin anabolism, sterigmatocystin biosynthesis, sterigmatocystin formation, sterigmatocystin synthesis Relationships: is a type of toxin biosynthetic process [GO:0009403]; is a type of sterigmatocystin metabolic process [GO:0045460] Regulation: regulated by regulation of sterigmatocystin biosynthetic process [GO:0010913]; positively regulated by positive regulation of sterigmatocystin biosynthetic process [GO:0010914]; negatively regulated by negative regulation of sterigmatocystin biosynthetic process [GO:1900760] References: PMID:10618248